toluene 2-monooxygenase activity [GO:0018644] (molecular function) Definition: Catalysis of the reaction: toluene + H+ + NADH + O2 = 2-hydroxytoluene + H2O + NAD+. Relationships: is a type of oxidoreductase activity, acting on paired donors, with incorporation or reduction of molecular oxygen, NAD(P)H as one donor, and incorporation of one atom of oxygen [GO:0016709] Sources: RHEA:20349